{
  "term_label": "sialic acid binding",
  "gene_name": "Sialic acid-binding Ig-like lectin 7",
  "term_id": "GO:0033691",
  "gene": "UniProtKB:Q9Y286",
  "gene_symbol": "SIGLEC7"
}